{
  "gene_symbol": "CD300LD",
  "term_id": "GO:0005886",
  "term_label": "plasma membrane",
  "gene": "UniProtKB:Q6UXZ3",
  "gene_name": "CMRF35-like molecule 5"
}